{
  "gene": "UniProtKB:Q15038",
  "term_id": "UNKNOWN:0002",
  "gene_name": "DAZ-associated protein 2",
  "gene_symbol": "DAZAP2",
  "term_label": "Unknown biological process"
}